{
  "term_id": "UNKNOWN:0001",
  "gene_name": "Myotubularin-related protein 10",
  "gene": "UniProtKB:Q9NXD2",
  "term_label": "Unknown molecular function",
  "gene_symbol": "MTMR10"
}